{
  "gene": "UniProtKB:Q96GZ6",
  "term_id": "UNKNOWN:0001",
  "gene_symbol": "SLC41A3",
  "gene_name": "Solute carrier family 41 member 3",
  "term_label": "Unknown molecular function"
}